{
  "term_id": "GO:1990756",
  "term_label": "ubiquitin-like ligase-substrate adaptor activity",
  "gene": "UniProtKB:O60811",
  "gene_symbol": "PRAMEF2",
  "gene_name": "PRAME family member 2"
}